{
  "gene_symbol": "PROX2",
  "gene": "UniProtKB:Q3B8N5",
  "term_label": "regulation of transcription by RNA polymerase II",
  "term_id": "GO:0006357",
  "gene_name": "Prospero homeobox protein 2"
}